{
  "term_id": "GO:0008023",
  "gene": "UniProtKB:Q96CJ1",
  "gene_symbol": "EAF2",
  "gene_name": "ELL-associated factor 2",
  "term_label": "transcription elongation factor complex"
}